negative regulation of protein sumoylation [GO:0033234] (biological process) Also known as: negative regulation of sumoylation Definition: Any process that stops, prevents, or reduces the frequency, rate or extent of the addition of SUMO groups to a protein. Sources: GOC:mah Relationships: is a type of regulation of protein sumoylation [GO:0033233]; is a type of GO:1903321; RO_0002212 protein sumoylation [GO:0016925]